{
  "gene": "UniProtKB:Q9UJT2",
  "gene_name": "Testis-specific serine kinase substrate",
  "term_label": "centriole",
  "term_id": "GO:0005814",
  "gene_symbol": "TSKS"
}